{
  "gene": "UniProtKB:O94763",
  "gene_name": "Unconventional prefoldin RPB5 interactor 1",
  "term_id": "GO:0003714",
  "gene_symbol": "URI1",
  "term_label": "transcription corepressor activity"
}